{
  "term_id": "GO:0005634",
  "term_label": "nucleus",
  "gene_symbol": "TSPY3",
  "gene": "UniProtKB:P0CV98",
  "gene_name": "Testis-specific Y-encoded protein 3"
}